wing cell fate specification [GO:0035311] (biological process) References: PMID:10860999 Relationships: is_a GO:0060573; is part of wing and notum subfield formation [GO:0035309] Definition: The process in which a cell in the larval wing imaginal disc becomes capable of differentiating autonomously into a wing cell, if left in its normal environment.